{
  "term_label": "Unknown cellular component",
  "gene": "UniProtKB:A6NCL7",
  "gene_name": "Ankyrin repeat domain-containing protein 33B",
  "gene_symbol": "ANKRD33B",
  "term_id": "UNKNOWN:0003"
}